L-tryptophan biosynthetic process [GO:0000162] (BP) Sources: GOC:mah, ISBN:0471331309, MetaCyc:TRPSYN-PWY Also known as: L-tryptophan anabolism, L-tryptophan biosynthesis, aromatic amino acid family biosynthetic process, anthranilate pathway, tryptophan formation, tryptophan biosynthetic process, tryptophan synthesis Definition: The chemical reactions and pathways resulting in the formation of L-tryptophan, the chiral amino acid 2-amino-3-(1H-indol-3-yl)propanoic acid; L-tryptophan is synthesized from chorismate via anthranilate. Relationships: is_a L-tryptophan metabolic process [GO:0006568]; is a type of aromatic amino acid family biosynthetic process [GO:0009073]; is a type of indolalkylamine biosynthetic process [GO:0046219]; is a type of L-amino acid biosynthetic process [GO:0170034]; is a type of GO:0170038